{
  "gene": "UniProtKB:Q13905",
  "gene_symbol": "RAPGEF1",
  "term_id": "GO:0010976",
  "gene_name": "Rap guanine nucleotide exchange factor 1",
  "term_label": "positive regulation of neuron projection development"
}